{
  "gene_symbol": "ARPC1B",
  "term_label": "Arp2/3 complex-mediated actin nucleation",
  "gene_name": "Actin-related protein 2_3 complex subunit 1B",
  "gene": "UniProtKB:O15143",
  "term_id": "GO:0034314"
}